glucosaminyl-phosphatidylinositol O-acyltransferase activity [GO:0032216] (molecular function) Relationships: is a type of O-acyltransferase activity [GO:0008374] Also known as: glucosaminyl-phosphotidylinositol O-acyltransferase activity, GPI-inositol acyltransferase Definition: Catalysis of the reaction: 6-(alpha-D-glucosaminyl)-1-(1,2-diacyl-sn-glycero-3-phospho)-1D-myo-inositol + fatty acyl-CoA = 2-acyl-6-(alpha-D-glucosaminyl)-1-(1,2-diacyl-sn-glycero-3-phospho)-1D-myo-inositol + CoA. References: PMID:29484956 Sources: RHEA:60496